{
  "gene": "UniProtKB:Q8N5J2",
  "gene_name": "Ubiquitin carboxyl-terminal hydrolase MINDY-1",
  "gene_symbol": "MINDY1",
  "term_id": "UNKNOWN:0002",
  "term_label": "Unknown biological process"
}